{
  "gene_name": "Syntaxin-11",
  "gene": "UniProtKB:O75558",
  "term_id": "GO:0031201",
  "term_label": "SNARE complex",
  "gene_symbol": "STX11"
}